{
  "gene_symbol": "NUDT17",
  "term_id": "GO:0005777",
  "gene_name": "Nucleoside diphosphate-linked moiety X motif 17",
  "term_label": "peroxisome",
  "gene": "UniProtKB:P0C025"
}